negative regulation of uredospore formation [GO:0075254] (biological process) Relationships: is a type of negative regulation of asexual sporulation resulting in formation of a cellular spore [GO:0043944]; is a type of regulation of uredospore formation [GO:0075252]; negatively regulates uredospore formation [GO:0075251] Definition: Any process that stops, prevents, or reduces the frequency, rate or extent of uredospore formation, a process in which an asexual, dikaryotic, often rusty-colored spore, is formed in a structure called a uredinium. Sources: GOC:pamgo_curators Also known as: negative regulation of ureidospore formation